branched-chain amino acid transmembrane transporter activity [GO:0015658] (molecular function) Sources: GOC:ai, GOC:bf, GOC:mtg_transport, ISBN:0815340729 Definition: Enables the transfer of branched-chain amino acids from one side of a membrane to the other. Branched-chain amino acids are amino acids with a branched carbon skeleton without rings. Subtypes: L-valine transmembrane transporter activity [GO:0005304], L-isoleucine transmembrane transporter activity [GO:0015188], L-leucine transmembrane transporter activity [GO:0015190], branched-chain amino acid:sodium symporter activity [GO:0015657] Also known as: branched-chain aliphatic amino acid transmembrane transporter activity, branched-chain aliphatic amino acid transporter activity, leucine/valine/isoleucine permease activity, valine/tyrosine/tryptophan permease activity Relationships: is a type of GO:0046943; is part of branched-chain amino acid transport [GO:0015803]